activation of microtubule nucleation [GO:0090064] (biological process) Relationships: is a type of GO:0090063 Definition: Any process that starts the inactive process of microtubule nucleation. Microtubule nucleation is the 'de novo' formation of a microtubule, in which tubulin heterodimers form metastable oligomeric aggregates, some of which go on to support formation of a complete microtubule. Microtubule nucleation usually occurs from a specific site within a cell. Sources: GOC:dph, GOC:tb